{
  "term_label": "nucleus",
  "gene_name": "Non-histone chromosomal protein HMG-17",
  "term_id": "GO:0005634",
  "gene_symbol": "HMGN2",
  "gene": "UniProtKB:P05204"
}